positive regulation of anti-Mullerian hormone signaling pathway [GO:1902614] (biological process) Definition: Any process that activates or increases the frequency, rate or extent of anti-Mullerian hormone signaling pathway. References: PMID:23624077 Sources: GOC:TermGenie, GOC:hjd, GO_REF:0000058 Also known as: up regulation of anti-Mullerian hormone signaling pathway, up-regulation of anti-Mullerian hormone signaling pathway, upregulation of anti-Mullerian hormone signaling pathway, activation of anti-Mullerian hormone signaling pathway Relationships: is a type of positive regulation of transmembrane receptor protein serine/threonine kinase signaling pathway [GO:0090100]; is a type of regulation of anti-Mullerian hormone signaling pathway [GO:1902612]; positively regulates anti-Mullerian hormone receptor signaling pathway [GO:1990262]